protein-glutamine glutaminase activity [GO:0050568] (molecular function) Also known as: destabilase activity, glutaminyl-peptide glutaminase activity, glutaminylpeptide glutaminase activity, peptidoglutaminase II activity, peptidylglutaminase II, protein-L-glutamine amidohydrolase activity Definition: Catalysis of the reaction: protein L-glutamine + H2O = protein L-glutamate + NH3. Relationships: is a type of hydrolase activity, acting on carbon-nitrogen (but not peptide) bonds, in linear amides [GO:0016811]; is a type of catalytic activity, acting on a protein [GO:0140096] Sources: EC:3.5.1.44, MetaCyc:CHEBDEAMID-RXN